{
  "term_label": "Unknown cellular component",
  "term_id": "UNKNOWN:0003",
  "gene_symbol": "FAM162B",
  "gene": "UniProtKB:Q5T6X4",
  "gene_name": "Protein FAM162B"
}